{
  "term_label": "peptidyl-prolyl cis-trans isomerase activity",
  "gene": "UniProtKB:Q13451",
  "gene_symbol": "FKBP5",
  "term_id": "GO:0003755",
  "gene_name": "Peptidyl-prolyl cis-trans isomerase FKBP5"
}